{
  "gene_symbol": "MYPN",
  "gene_name": "Myopalladin",
  "gene": "UniProtKB:Q86TC9",
  "term_label": "Z disc",
  "term_id": "GO:0030018"
}